{
  "gene_name": "Proliferating cell nuclear antigen",
  "gene": "UniProtKB:P12004",
  "term_id": "GO:0006272",
  "term_label": "leading strand elongation",
  "gene_symbol": "PCNA"
}